{
  "gene": "UniProtKB:Q14517",
  "gene_symbol": "FAT1",
  "term_label": "adherens junction",
  "gene_name": "Protocadherin Fat 1",
  "term_id": "GO:0005912"
}